{
  "gene_symbol": "BRAF",
  "term_id": "GO:0005737",
  "term_label": "cytoplasm",
  "gene_name": "Serine_threonine-protein kinase B-raf",
  "gene": "UniProtKB:P15056"
}